{
  "term_id": "GO:0043527",
  "gene": "UniProtKB:Q9UBP6",
  "gene_name": "tRNA (guanine-N(7)-)-methyltransferase",
  "gene_symbol": "METTL1",
  "term_label": "tRNA methyltransferase complex"
}